{
  "gene": "UniProtKB:Q14807",
  "gene_name": "Kinesin-like protein KIF22",
  "term_label": "kinesin complex",
  "gene_symbol": "KIF22",
  "term_id": "GO:0005871"
}